{
  "gene": "UniProtKB:Q92886",
  "term_label": "E-box binding",
  "term_id": "GO:0070888",
  "gene_name": "Neurogenin-1",
  "gene_symbol": "NEUROG1"
}